detection of stimulus [GO:0051606] (biological process) Subtypes: GO:0009581, detection of abiotic stimulus [GO:0009582], detection of chemical stimulus [GO:0009593], detection of biotic stimulus [GO:0009595], detection of inactivity [GO:0014863], detection of activity [GO:0014865], GO:0050906 Relationships: is a type of response to stimulus [GO:0050896] Also known as: stimulus detection, perception of stimulus, stimulus sensing Definition: The series of events in which a stimulus is received by a cell or organism and converted into a molecular signal. Sources: GOC:add, GOC:ai, GOC:dph, GOC:mah